{
  "gene": "UniProtKB:Q8IZP0",
  "term_label": "cell projection morphogenesis",
  "term_id": "GO:0048858",
  "gene_symbol": "ABI1",
  "gene_name": "Abl interactor 1"
}